{
  "gene": "UniProtKB:Q9Y4E5",
  "term_id": "GO:0061665",
  "gene_name": "E3 SUMO-protein ligase ZNF451",
  "term_label": "SUMO ligase activity",
  "gene_symbol": "ZNF451"
}